{
  "term_label": "intracellular cyclic nucleotide activated cation channel complex",
  "gene_symbol": "CNGA2",
  "gene": "UniProtKB:Q16280",
  "term_id": "GO:0017071",
  "gene_name": "Cyclic nucleotide-gated olfactory channel"
}